{
  "gene_symbol": "TNN",
  "gene_name": "Tenascin-N",
  "gene": "UniProtKB:Q9UQP3",
  "term_id": "GO:1990138",
  "term_label": "neuron projection extension"
}